imidazoleglycerol-phosphate synthase activity [GO:0000107] (molecular function) Sources: RHEA:24793 Relationships: is_a GO:0016763 Definition: Catalysis of the reaction: phosphoribulosylformimino-AICAR-P + L-glutamine = D-erythro-imidazole-glycerol-phosphate + aminoimidazole carboxamide ribonucleotide + L-glutamate + 2 H+. Also known as: glutamine amidotransferase:cyclase activity, imidazole glycerol phosphate synthase activity, imidazoleglycerol phosphate synthase activity, imidazole-glycerol-phosphate synthase activity